{
  "gene": "UniProtKB:H3BTG2",
  "term_id": "UNKNOWN:0001",
  "gene_symbol": "TEX46",
  "gene_name": "Testis-expressed protein 46",
  "term_label": "Unknown molecular function"
}